{
  "term_id": "GO:1905289",
  "term_label": "regulation of CAMKK-AMPK signaling cascade",
  "gene_name": "Huntingtin",
  "gene": "UniProtKB:P42858",
  "gene_symbol": "HTT"
}